{
  "gene_symbol": "CDC25C",
  "term_id": "GO:0000086",
  "gene_name": "M-phase inducer phosphatase 3",
  "term_label": "G2/M transition of mitotic cell cycle",
  "gene": "UniProtKB:P30307"
}